{
  "term_label": "potassium ion leak channel activity",
  "gene_symbol": "KCNK5",
  "gene": "UniProtKB:O95279",
  "gene_name": "Potassium channel subfamily K member 5",
  "term_id": "GO:0022841"
}